negative regulation of anterior neural cell fate commitment of the neural plate by fibroblast growth factor receptor signaling pathway [GO:0022003] (biological process) Also known as: fgf receptor signaling involved in down regulation of anterior neural cell fate of the neural plate, fgf receptor signaling involved in down-regulation of anterior neural cell fate of the neural plate, fgf receptor signaling involved in downregulation of anterior neural cell fate of the neural plate, fgf receptor signaling involved in negative regulation of anterior neural cell fate of the neural plate, fgf receptor signalling involved in negative regulation of anterior neural cell fate of the neural plate, fgf receptor signaling involved in inhibition of anterior neural cell fate of the neural plate Relationships: is a type of GO:0022001; is a type of fibroblast growth factor receptor signaling pathway involved in neural plate anterior/posterior pattern formation [GO:0060825] Definition: The series of molecular signals that stops, prevents or reduces the frequency or rate at which cell adopts an anterior neural cell fate, generated as a consequence of a fibroblast growth factor receptor binding to one of its physiological ligands. Sources: GOC:cls, GOC:dgh, GOC:dph, GOC:jid, GOC:tb